{
  "term_id": "UNKNOWN:0003",
  "gene": "UniProtKB:Q9GZW5",
  "gene_symbol": "SCAND2P",
  "gene_name": "Putative SCAN domain-containing protein SCAND2P",
  "term_label": "Unknown cellular component"
}